{
  "term_id": "GO:0004674",
  "gene_name": "Serine_threonine-protein kinase N2",
  "gene_symbol": "PKN2",
  "term_label": "protein serine/threonine kinase activity",
  "gene": "UniProtKB:Q16513"
}